{
  "gene": "UniProtKB:Q8TBY9",
  "gene_name": "Cilia- and flagella-associated protein 251",
  "term_id": "UNKNOWN:0002",
  "gene_symbol": "CFAP251",
  "term_label": "Unknown biological process"
}